{
  "gene_symbol": "SLC5A3",
  "gene_name": "Sodium_myo-inositol cotransporter",
  "term_label": "myo-inositol:sodium symporter activity",
  "term_id": "GO:0005367",
  "gene": "UniProtKB:P53794"
}